{
  "gene": "UniProtKB:P34972",
  "gene_symbol": "CNR2",
  "term_id": "GO:0005737",
  "term_label": "cytoplasm",
  "gene_name": "Cannabinoid receptor 2"
}